extracellular matrix binding [GO:0050840] (molecular function) Also known as: extracellular matrix constituent binding, adhesive extracellular matrix constituent Relationships: is a type of binding [GO:0005488] Definition: Binding to a component of the extracellular matrix. Subtypes: laminin binding [GO:0043236], GO:0044730, host cell extracellular matrix binding [GO:0046810], GO:0050436, GO:0098633 Sources: GOC:ai